{
  "gene_symbol": "RPS2",
  "term_label": "translation",
  "term_id": "GO:0006412",
  "gene_name": "Small ribosomal subunit protein uS5",
  "gene": "UniProtKB:P15880"
}